{
  "term_label": "regulation of systemic arterial blood pressure by endothelin",
  "gene_symbol": "EDN1",
  "gene": "UniProtKB:P05305",
  "term_id": "GO:0003100",
  "gene_name": "Endothelin-1"
}